{
  "gene_symbol": "RLN1",
  "gene": "UniProtKB:P04808",
  "term_label": "Unknown cellular component",
  "gene_name": "Prorelaxin H1",
  "term_id": "UNKNOWN:0003"
}